{
  "gene_symbol": "POLR1G",
  "gene_name": "DNA-directed RNA polymerase I subunit RPA34",
  "gene": "UniProtKB:O15446",
  "term_label": "Unknown molecular function",
  "term_id": "UNKNOWN:0001"
}